{
  "gene_name": "CTP synthase 2",
  "gene": "UniProtKB:Q9NRF8",
  "term_label": "CTP synthase activity",
  "term_id": "GO:0003883",
  "gene_symbol": "CTPS2"
}